{
  "term_id": "GO:0051016",
  "gene": "UniProtKB:P35612",
  "gene_name": "Beta-adducin",
  "term_label": "barbed-end actin filament capping",
  "gene_symbol": "ADD2"
}